{
  "gene": "UniProtKB:P15812",
  "gene_symbol": "CD1E",
  "gene_name": "T-cell surface glycoprotein CD1e, membrane-associated",
  "term_id": "GO:0030884",
  "term_label": "exogenous lipid antigen binding"
}